{
  "term_label": "N-box binding",
  "gene_symbol": "HES1",
  "gene_name": "Transcription factor HES-1",
  "term_id": "GO:0071820",
  "gene": "UniProtKB:Q14469"
}